{
  "term_id": "GO:0030183",
  "term_label": "B cell differentiation",
  "gene_symbol": "CD79A",
  "gene": "UniProtKB:P11912",
  "gene_name": "B-cell antigen receptor complex-associated protein alpha chain"
}